{
  "gene_name": "Ubiquinol-cytochrome-c reductase complex assembly factor 3",
  "gene_symbol": "UQCC3",
  "term_label": "mitochondrial electron transport, ubiquinol to cytochrome c",
  "term_id": "GO:0006122",
  "gene": "UniProtKB:Q6UW78"
}